{
  "gene_name": "P2X purinoceptor 6",
  "term_label": "extracellularly ATP-gated monoatomic cation channel activity",
  "gene_symbol": "P2RX6",
  "term_id": "GO:0004931",
  "gene": "UniProtKB:O15547"
}